{
  "gene_name": "Gamma-aminobutyric acid receptor subunit beta-2",
  "term_id": "GO:0005254",
  "gene": "UniProtKB:P47870",
  "term_label": "chloride channel activity",
  "gene_symbol": "GABRB2"
}